{
  "term_label": "aldose reductase (NADPH) activity",
  "gene_name": "Aldo-keto reductase family 1 member B1",
  "gene": "UniProtKB:P15121",
  "term_id": "GO:0004032",
  "gene_symbol": "AKR1B1"
}